{
  "gene": "UniProtKB:Q00973",
  "gene_symbol": "B4GALNT1",
  "term_id": "GO:0008376",
  "gene_name": "Beta-1,4 N-acetylgalactosaminyltransferase 1",
  "term_label": "acetylgalactosaminyltransferase activity"
}